{
  "term_label": "intracellular calcium ion homeostasis",
  "term_id": "GO:0006874",
  "gene_symbol": "PTH1R",
  "gene_name": "Parathyroid hormone_parathyroid hormone-related peptide receptor",
  "gene": "UniProtKB:Q03431"
}